{
  "term_label": "negative regulation of telomere maintenance via recombination",
  "term_id": "GO:0032208",
  "gene_name": "Telomeric repeat-binding factor 2",
  "gene": "UniProtKB:Q15554",
  "gene_symbol": "TERF2"
}